cellular response to oxygen levels [GO:0071453] (biological process) Also known as: cellular response to oxygen Subtypes: GO:0036294, cellular response to increased oxygen levels [GO:0036295] Sources: GOC:mah Relationships: is_a response to oxygen levels [GO:0070482]; is a type of cellular response to chemical stimulus [GO:0070887] Definition: Any process that results in a change in state or activity of a cell (in terms of movement, secretion, enzyme production, gene expression, etc.) as a result of a stimulus reflecting the presence, absence, or concentration of oxygen.